{
  "gene": "UniProtKB:P62495",
  "gene_symbol": "ETF1",
  "term_id": "GO:0016149",
  "gene_name": "Eukaryotic peptide chain release factor subunit 1",
  "term_label": "translation release factor activity, codon specific"
}